adrenomedullin receptor activity [GO:0001605] (molecular function) Definition: Combining with adrenomedullin to initiate a change in cell activity. Sources: GOC:ai Also known as: G10D receptor Relationships: is_a calcitonin family receptor activity [GO:0097642]